{
  "gene": "UniProtKB:Q9UGC6",
  "gene_symbol": "RGS17",
  "term_label": "GTPase activator activity",
  "gene_name": "Regulator of G-protein signaling 17",
  "term_id": "GO:0005096"
}